{
  "term_label": "RNA polymerase II cis-regulatory region sequence-specific DNA binding",
  "gene": "UniProtKB:Q01167",
  "gene_symbol": "FOXK2",
  "gene_name": "Forkhead box protein K2",
  "term_id": "GO:0000978"
}